{
  "term_label": "vacuolar proton-transporting V-type ATPase, V1 domain",
  "term_id": "GO:0000221",
  "gene_name": "V-type proton ATPase subunit C 2",
  "gene": "UniProtKB:Q8NEY4",
  "gene_symbol": "ATP6V1C2"
}